{
  "gene_symbol": "PARD6G",
  "gene": "UniProtKB:Q9BYG4",
  "term_label": "apical plasma membrane",
  "term_id": "GO:0016324",
  "gene_name": "Partitioning defective 6 homolog gamma"
}